{
  "gene_name": "Tyrosine-protein kinase Fer",
  "term_label": "plasma membrane",
  "gene": "UniProtKB:P16591",
  "term_id": "GO:0005886",
  "gene_symbol": "FER"
}